{
  "gene_symbol": "EXOC3-AS1",
  "gene_name": "Uncharacterized protein EXOC3-AS1",
  "term_id": "UNKNOWN:0001",
  "term_label": "Unknown molecular function",
  "gene": "UniProtKB:Q8N2X6"
}